{
  "term_label": "NSL complex",
  "gene_symbol": "KANSL2",
  "gene": "UniProtKB:Q9H9L4",
  "gene_name": "KAT8 regulatory NSL complex subunit 2",
  "term_id": "GO:0044545"
}